{
  "term_id": "GO:0005634",
  "gene_name": "Insulinoma-associated protein 2",
  "gene": "UniProtKB:Q96T92",
  "gene_symbol": "INSM2",
  "term_label": "nucleus"
}